{
  "gene": "UniProtKB:Q14512",
  "gene_name": "Fibroblast growth factor-binding protein 1",
  "term_id": "GO:0007267",
  "gene_symbol": "FGFBP1",
  "term_label": "cell-cell signaling"
}